{
  "term_label": "Unknown molecular function",
  "gene_symbol": "VCX3A",
  "term_id": "UNKNOWN:0001",
  "gene": "UniProtKB:Q9NNX9",
  "gene_name": "Variable charge X-linked protein 3"
}